{
  "gene": "UniProtKB:A0A8Q3SIG1",
  "gene_name": "Vitellogenin domain-containing protein",
  "term_id": "UNKNOWN:0003",
  "term_label": "Unknown cellular component",
  "gene_symbol": "LOC400499"
}